{
  "gene_symbol": "HNF1A",
  "gene_name": "Hepatocyte nuclear factor 1-alpha",
  "term_id": "GO:0006357",
  "term_label": "regulation of transcription by RNA polymerase II",
  "gene": "UniProtKB:P20823"
}